{
  "gene_symbol": "TMEM204",
  "gene_name": "Transmembrane protein 204",
  "term_label": "Unknown molecular function",
  "gene": "UniProtKB:Q9BSN7",
  "term_id": "UNKNOWN:0001"
}